cholesterol monooxygenase (side-chain-cleaving) activity [GO:0008386] (molecular function) Also known as: steroid 20-22 desmolase activity, steroid 20-22-lyase activity, Cyp11a1, cytochrome P-450(scc) activity, cytochrome p450(scc) activity, C27-side chain cleavage enzyme, cholesterol 20-22-desmolase activity, cholesterol C(20-22) desmolase activity, cholesterol C20-22 desmolase activity, cholesterol desmolase activity, cholesterol side-chain cleavage enzyme activity, cholesterol side-chain-cleaving enzyme activity, cholesterol,reduced-adrenal-ferredoxin:oxygen oxidoreductase (side-chain-cleaving), cytochrome P-450scc, cytochrome p450scc, desmolase, steroid 20-22, enzymes, cholesterol side-chain-cleaving Sources: EC:1.14.15.6 Relationships: is a type of GO:0008395; is a type of oxidoreductase activity, acting on paired donors, with incorporation or reduction of molecular oxygen, reduced iron-sulfur protein as one donor, and incorporation of one atom of oxygen [GO:0016713] Definition: Catalysis of the reaction: cholesterol + reduced adrenal ferredoxin + O2 = pregnenolone + 4-methylpentanal + oxidized adrenal ferredoxin + H2O.